{
  "gene": "UniProtKB:Q8N594",
  "gene_name": "MPN domain-containing protein",
  "gene_symbol": "MPND",
  "term_id": "GO:0008237",
  "term_label": "metallopeptidase activity"
}